{
  "term_label": "Unknown molecular function",
  "term_id": "UNKNOWN:0001",
  "gene_symbol": "RTL1",
  "gene_name": "Retrotransposon-like protein 1",
  "gene": "UniProtKB:A6NKG5"
}